(R)-carnitine transmembrane transporter activity [GO:1901235] (molecular function) Definition: Enables the transfer of (R)-carnitine from one side of a membrane to the other. Relationships: is a type of carnitine transmembrane transporter activity [GO:0015226]; is part of (R)-carnitine transmembrane transport [GO:1902270] Subtypes: (R)-carnitine:4-(trimethylammonio)butanoate antiporter activity [GO:0044667] References: PMID:16365042, PMID:20357772, PMID:20829798 Sources: GOC:TermGenie